{
  "gene_name": "Metastasis-associated protein MTA1",
  "gene_symbol": "MTA1",
  "term_label": "response to ionizing radiation",
  "gene": "UniProtKB:Q13330",
  "term_id": "GO:0010212"
}